{
  "gene_name": "Transcriptional regulator PINT87aa",
  "gene_symbol": "LINC-PINT",
  "gene": "UniProtKB:A0A455ZAR2",
  "term_label": "Unknown molecular function",
  "term_id": "UNKNOWN:0001"
}